farnesoic acid O-methyltransferase activity [GO:0019010] (molecular function) References: PMID:12135499, PMID:14530389, PMID:18549957 Sources: EC:2.1.1.325 Definition: Catalysis of the reaction: (2E,6E)-farnesoate + S-adenosyl-L-methionine = methyl (2E,6E)-farnesoate + S-adenosyl-L-homocysteine. Also converts juvenile hormone III carboxylate into juvenile hormone-III. Also known as: S-adenosyl-methionine:farnesoic acid O-methyltransferase activity, juvenile hormone acid methyltransferase activity, juvenile hormone-III synthase activity Relationships: is a type of O-methyltransferase activity [GO:0008171]; is a type of S-adenosylmethionine-dependent methyltransferase activity [GO:0008757]